negative regulation of macrophage differentiation [GO:0045650] (biological process) Sources: GOC:go_curators Relationships: is a type of negative regulation of myeloid leukocyte differentiation [GO:0002762]; is a type of GO:0045649; negatively regulates macrophage differentiation [GO:0030225] Also known as: down regulation of macrophage differentiation, down-regulation of macrophage differentiation, downregulation of macrophage differentiation, inhibition of macrophage differentiation Subtypes: GO:0014007 Definition: Any process that stops, prevents, or reduces the frequency, rate or extent of macrophage differentiation.